{
  "gene": "UniProtKB:Q9HAZ1",
  "gene_name": "Dual specificity protein kinase CLK4",
  "term_label": "protein serine/threonine kinase activity",
  "term_id": "GO:0004674",
  "gene_symbol": "CLK4"
}